cerebellar cortex structural organization [GO:0021698] (biological process) Relationships: is a type of anatomical structure arrangement [GO:0048532]; is part of cerebellar cortex morphogenesis [GO:0021696] Definition: The process that contributes to the act of creating the structural organization of the cerebellar cortex. This process pertains to the physical shaping of a rudimentary structure. The cerebellar cortex is a thin mantle of gray matter that covers the surface of each cerebral hemisphere. It has a characteristic morphology with convolutions (gyri) and crevices (sulci) that have specific functions. Six layers of nerve cells and the nerve pathways that connect them comprise the cerebellar cortex. Together, these regions are responsible for the processes of conscious thought, perception, emotion and memory as well as advanced motor function. Also known as: cerebellar cortex structural organisation Sources: GOC:cls, GOC:dgh, GOC:dph, GOC:jid, GO_REF:0000021